regulation of mRNA 3'-end processing [GO:0031440] (biological process) Relationships: is a type of GO:0050684; regulates mRNA 3'-end processing [GO:0031124] Sources: GOC:mah Subtypes: negative regulation of mRNA 3'-end processing [GO:0031441], positive regulation of mRNA 3'-end processing [GO:0031442], regulation of mRNA alternative polyadenylation [GO:0140408] Definition: Any process that modulates the frequency, rate or extent of mRNA 3'-end processing, any process involved in forming the mature 3' end of an mRNA molecule.